{
  "gene": "UniProtKB:Q8WU10",
  "term_id": "UNKNOWN:0001",
  "term_label": "Unknown molecular function",
  "gene_name": "Pyridine nucleotide-disulfide oxidoreductase domain-containing protein 1",
  "gene_symbol": "PYROXD1"
}